{
  "gene_name": "Dihydrofolate reductase",
  "term_id": "GO:0046654",
  "gene": "UniProtKB:P00374",
  "gene_symbol": "DHFR",
  "term_label": "tetrahydrofolate biosynthetic process"
}